{
  "gene_name": "Contactin-1",
  "gene": "UniProtKB:Q12860",
  "term_id": "GO:0098632",
  "term_label": "cell-cell adhesion mediator activity",
  "gene_symbol": "CNTN1"
}